{
  "gene_name": "Olfactory receptor 51E1",
  "gene_symbol": "OR51E1",
  "term_id": "UNKNOWN:0002",
  "gene": "UniProtKB:Q8TCB6",
  "term_label": "Unknown biological process"
}